{
  "gene_symbol": "OR8B8",
  "term_id": "GO:0007186",
  "term_label": "G protein-coupled receptor signaling pathway",
  "gene_name": "Olfactory receptor 8B8",
  "gene": "UniProtKB:Q15620"
}